{
  "gene_symbol": "PNPLA2",
  "term_id": "GO:0019433",
  "gene_name": "Patatin-like phospholipase domain-containing protein 2",
  "gene": "UniProtKB:Q96AD5",
  "term_label": "triglyceride catabolic process"
}